lung basal cell differentiation [GO:0060508] (biological process) Sources: GOC:dph, GOC:mtg_lung Relationships: is a type of lung cell differentiation [GO:0060479]; is part of lung epithelium development [GO:0060428] Definition: The process in which relatively unspecialized cells, e.g. embryonic or regenerative cells, acquire specialized structural and/or functional features of a mature basal cell found in the lung. Differentiation includes the processes involved in commitment of a cell to a specific fate. A basal cell is an epithelial stem cell. Also known as: pulmonary basal cell differentiation